positive regulation of transmembrane transport [GO:0034764] (biological process) Definition: Any process that activates or increases the frequency, rate or extent of the directed movement of a solute from one side of a membrane to the other. Subtypes: positive regulation of L-glutamate import across plasma membrane [GO:0002038], GO:0010747, positive regulation of D-glucose transmembrane transport [GO:0010828], positive regulation of monoatomic ion transmembrane transport [GO:0034767], GO:0035432, positive regulation of glycerol transport [GO:0090372], positive regulation of D-aspartate import across plasma membrane [GO:0140217], GO:1900072, positive regulation of glycine import across plasma membrane [GO:1900925], positive regulation of L-threonine import across plasma membrane [GO:1900928], positive regulation of L-tyrosine import across plasma membrane [GO:1900931], GO:1901036, GO:1902269, positive regulation of (R)-carnitine transmembrane transport [GO:1902274], GO:1902836, positive regulation of protein import into chloroplast stroma [GO:1904216], positive regulation of L-lysine import across plasma membrane [GO:1905010], positive regulation of uracil import across plasma membrane [GO:1905531], positive regulation of L-leucine import across plasma membrane [GO:1905534], positive regulation of L-arginine import across plasma membrane [GO:1905589], positive regulation of L-methionine import across plasma membrane [GO:1905626], positive regulation of xenobiotic detoxification by transmembrane export across the plasma membrane [GO:1905701], positive regulation of phosphate transmembrane transport [GO:2000187], positive regulation of dipeptide transmembrane transport [GO:2001150] Sources: GOC:mah Also known as: positive regulation of membrane transport, up regulation of transmembrane transport, up-regulation of transmembrane transport, upregulation of transmembrane transport, activation of transmembrane transport, stimulation of transmembrane transport Relationships: is a type of regulation of transmembrane transport [GO:0034762]; is a type of positive regulation of cellular process [GO:0048522]; is a type of positive regulation of transport [GO:0051050]; positively regulates transmembrane transport [GO:0055085]